{
  "gene": "UniProtKB:P15421",
  "gene_symbol": "GYPE",
  "term_id": "UNKNOWN:0002",
  "gene_name": "Glycophorin-E",
  "term_label": "Unknown biological process"
}